basal RNA polymerase II transcription machinery binding [GO:0001099] (molecular function) Sources: GOC:txnOH Definition: Binding to a component of the basal transcription machinery for RNA polymerase II which is composed of the RNA polymerase II core enzyme, a multisubunit eukaryotic nuclear RNA polymerase typically composed of twelve subunits, and the basal RNA polymerase II transcription factors, the minimal set of factors required for formation of the preinitiation complex (PIC) by the RNA polymerase. Subtypes: RNA polymerase II complex binding [GO:0000993], RNA polymerase II general transcription initiation factor binding [GO:0001091] Also known as: basal RNAP II transcription machinery binding Note: Note that the definition of basal, or general, transcription factors has typically been done at a small number of well characterized activator-independent promoters. At an activator-dependent promoter, one or more additional factors are generally required in addition to the basal factors. Relationships: is a type of basal transcription machinery binding [GO:0001098]